{
  "gene": "UniProtKB:P0C091",
  "gene_name": "FRAS1-related extracellular matrix protein 3",
  "gene_symbol": "FREM3",
  "term_label": "extracellular matrix",
  "term_id": "GO:0031012"
}